toxin sequestering activity [GO:0097351] (molecular function) References: PMID:19143615, PMID:19325885, PMID:21819231, PMID:22545240, PMID:24806488 Sources: GOC:rs, Wikipedia:Toxin-antitoxin_system#Type_II Relationships: is_a GO:0140313 Note: There may be more than one antitoxin to a toxic protein. Instances of this activity are known only in prokaryotes, where the toxic protein may be a ribonuclease, a DNA gyrase, or other. Definition: Binding to a toxin to prevent it from interacting with other partners or to inhibit its localization to the area of the cell or complex where it is active. Also known as: toxin-antitoxin pair type I binding, toxin-antitoxin pair type II binding